{
  "gene": "UniProtKB:Q7Z3C6",
  "term_label": "phospholipid scramblase activity",
  "gene_symbol": "ATG9A",
  "gene_name": "Autophagy-related protein 9A",
  "term_id": "GO:0017128"
}